{
  "term_id": "UNKNOWN:0003",
  "term_label": "Unknown cellular component",
  "gene_symbol": "POU2F3",
  "gene_name": "POU domain, class 2, transcription factor 3",
  "gene": "UniProtKB:Q9UKI9"
}